solute:proton symporter activity [GO:0015295] (molecular function) Definition: Enables the transfer of a solute or solutes from one side of a membrane to the other according to the reaction: solute(out) + H+(out) = solute(in) + H+(in). Sources: GOC:ai Also known as: solute:hydrogen symporter activity, L-idonate/D-gluconate:hydrogen symporter activity, heavy metal ion:hydrogen symporter activity, high affinity metal ion uptake transporter activity, low affinity metal ion uptake transporter activity, proline/glycine/betaine:hydrogen/sodium symporter activity Relationships: is a type of proton transmembrane transporter activity [GO:0015078]; is_a solute:monoatomic cation symporter activity [GO:0015294] Subtypes: GO:0005274, amino acid:proton symporter activity [GO:0005280], carbohydrate:proton symporter activity [GO:0005351], GO:0005352, GO:0005366, GO:0008512, nitrate:proton symporter activity [GO:0009671], GO:0009672, phosphate:proton symporter activity [GO:0015317], peptide:proton symporter activity [GO:0015333], GO:0015345, GO:0015346, acetate:proton symporter activity [GO:0015360], GO:0015366, potassium:proton symporter activity [GO:0015387], aromatic amino acid:proton symporter activity [GO:0015494], cytosine:proton symporter activity [GO:0015504], nucleoside:proton symporter activity [GO:0015506], citrate:proton symporter activity [GO:0015531], alpha-ketoglutarate:proton symporter activity [GO:0015532], shikimate:proton symporter activity [GO:0015533], sialic acid:proton symporter activity [GO:0015538], 3-hydroxyphenyl propionate:proton symporter activity [GO:0015540], GO:0015650, quaternary ammonium group:proton symporter activity [GO:0015652], thiamine:proton symporter activity [GO:0034215], GO:0090448, selenite:proton symporter activity [GO:0097079], succinate:proton symporter activity [GO:0097434], folic acid:proton symporter activity [GO:0140211]